substantia nigra development [GO:0021762] (biological process) Relationships: is_a neural nucleus development [GO:0048857]; BFO_0000050 midbrain development [GO:0030901] Sources: GOC:cls, GOC:dgh, GOC:dph, GOC:jid, GO_REF:0000021 Definition: The progression of the substantia nigra over time from its initial formation until its mature state. The substantia nigra is the layer of gray substance that separates the posterior parts of the cerebral peduncles (tegmentum mesencephali) from the anterior parts; it normally includes a posterior compact part with many pigmented cells (pars compacta) and an anterior reticular part whose cells contain little pigment (pars reticularis).